{
  "gene_name": "Threonine synthase-like 2",
  "term_id": "GO:0030170",
  "gene": "UniProtKB:Q86YJ6",
  "term_label": "pyridoxal phosphate binding",
  "gene_symbol": "THNSL2"
}